{
  "term_label": "histone binding",
  "gene_symbol": "PWWP2A",
  "gene": "UniProtKB:Q96N64",
  "gene_name": "PWWP domain-containing protein 2A",
  "term_id": "GO:0042393"
}